{
  "term_id": "GO:0061630",
  "term_label": "ubiquitin protein ligase activity",
  "gene_name": "E3 ubiquitin-protein ligase RNF13",
  "gene": "UniProtKB:O43567",
  "gene_symbol": "RNF13"
}